glucose dehydrogenase activity [GO:0004344] (molecular function) Definition: Catalysis of the reaction: D-glucose + acceptor = D-glucono-1,5-lactone + reduced acceptor. Relationships: is a type of GO:0016614 Also known as: glucose dehydrogenase (acceptor) activity, soluble glucose dehydrogenase References: PMID:22027299 Subtypes: quinoprotein glucose dehydrogenase activity [GO:0008876], GO:0047936, GO:0140762